{
  "gene_name": "Putative TAP2-associated 6.5 kDa polypeptide",
  "term_id": "UNKNOWN:0002",
  "term_label": "Unknown biological process",
  "gene_symbol": "Q9Y3F1",
  "gene": "UniProtKB:Q9Y3F1"
}